response to symbiont [GO:0009608] (biological process) Relationships: is a type of response to other organism [GO:0051707] Sources: GOC:hb, ISBN:0198506732 Definition: Any process that results in a change in state or activity of a cell or an organism (in terms of movement, secretion, enzyme production, gene expression, etc.) as a result of a stimulus from a symbiont, an organism living with an organism of a different species in close physical association. The symbiont is defined as the smaller of the organisms involved in a symbiotic interaction. Subtypes: response to parasitic plant [GO:0002241], detection of symbiont [GO:0009602], GO:0009609, GO:0009610, host response to induction by symbiont of tumor, nodule or growth in host [GO:0080034] Also known as: response of host to symbiont